{
  "term_label": "Unknown molecular function",
  "gene": "UniProtKB:Q8N806",
  "gene_symbol": "UBR7",
  "term_id": "UNKNOWN:0001",
  "gene_name": "Putative E3 ubiquitin-protein ligase UBR7"
}